{
  "term_label": "trans-Golgi network",
  "gene_symbol": "AP3M1",
  "gene": "UniProtKB:Q9Y2T2",
  "gene_name": "AP-3 complex subunit mu-1",
  "term_id": "GO:0005802"
}